{
  "gene_symbol": "PLEKHA7",
  "term_label": "pore complex",
  "gene": "UniProtKB:Q6IQ23",
  "term_id": "GO:0046930",
  "gene_name": "Pleckstrin homology domain-containing family A member 7"
}